{
  "term_label": "olfactory receptor activity",
  "gene_symbol": "OR1Q1",
  "gene": "UniProtKB:Q15612",
  "gene_name": "Olfactory receptor 1Q1",
  "term_id": "GO:0004984"
}